{
  "gene": "UniProtKB:Q8N6L1",
  "gene_name": "Keratinocyte-associated protein 2",
  "gene_symbol": "KRTCAP2",
  "term_label": "Unknown cellular component",
  "term_id": "UNKNOWN:0003"
}